hydroxymethylfurfural reductase (NADH) activity [GO:0033833] (molecular function) Definition: Catalysis of the reaction: 5-hydroxymethylfurfural + NADH + H+ = 2,5-bis-hydroxymethylfuran + NAD+. References: PMID:15338422, PMID:16652391 Sources: GOC:jp, GOC:mah Relationships: is a type of oxidoreductase activity, acting on the CH-OH group of donors, NAD or NADP as acceptor [GO:0016616]